NatC complex [GO:0031417] (cellular component) Definition: A conserved complex that catalyzes the transfer of an acetyl group to the N-terminal residue of a protein acceptor molecule that has a Met-Ile, Met-Leu, Met-Trp, or Met-Phe N-terminus. In Saccharomyces the complex includes Mak3p, Mak10p, and Mak31p. Also known as: N-terminal acetyltransferase C complex Relationships: is a type of N-terminal protein acetyltransferase complex [GO:0031414] References: PMID:12890471